plasma membrane organization [GO:0007009] (biological process) Relationships: is a type of membrane organization [GO:0061024]; is part of endomembrane system organization [GO:0010256] Sources: GOC:dph, GOC:jl, GOC:mah Regulation: regulated by GO:1903729 Subtypes: GO:0001778, plasma membrane phospholipid scrambling [GO:0017121], GO:0035045, myelin maintenance [GO:0043217], GO:0044856, plasma membrane fusion [GO:0045026], membrane reorganization involved in phagocytosis, engulfment [GO:0060098], GO:0097036, plasma membrane tubulation [GO:0097320], cornified envelope assembly [GO:1903575] Also known as: plasma membrane organisation, plasma membrane organization and biogenesis Definition: A process that is carried out at the cellular level which results in the assembly, arrangement of constituent parts, or disassembly of the plasma membrane.